{
  "gene_name": "Transcription cofactor vestigial-like protein 2",
  "gene_symbol": "VGLL2",
  "term_label": "Unknown molecular function",
  "term_id": "UNKNOWN:0001",
  "gene": "UniProtKB:Q8N8G2"
}